negative regulation of muscle cell chemotaxis toward tendon cell [GO:2001282] (BP) Definition: Any process that stops, prevents or reduces the frequency, rate or extent of the directed movement of a muscle cell towards a tendon cell in response to an external stimulus. For example, when the muscle cell arrives at the target tendon cell, migration is arrested so that attachments can be made between the cells. References: PMID:19793885, PMID:20404543 Sources: GOC:sart Also known as: negative regulation of muscle cell chemotaxis towards tendon cell, arrest of muscle cell chemotaxis, negative regulation of muscle cell attraction Relationships: is a type of negative regulation of cell migration [GO:0030336]; is_a negative regulation of chemotaxis [GO:0050922]; is a type of regulation of muscle cell chemotaxis toward tendon cell [GO:2001281]; negatively regulates muscle cell chemotaxis toward tendon cell [GO:0036061]